{
  "gene": "UniProtKB:P07203",
  "gene_name": "Glutathione peroxidase 1",
  "term_id": "GO:0042542",
  "gene_symbol": "GPX1",
  "term_label": "response to hydrogen peroxide"
}